{
  "gene_symbol": "MRPS28",
  "term_id": "GO:0005763",
  "term_label": "mitochondrial small ribosomal subunit",
  "gene_name": "Small ribosomal subunit protein bS1m",
  "gene": "UniProtKB:Q9Y2Q9"
}